{
  "gene_name": "3-ketodihydrosphingosine reductase",
  "term_id": "GO:0005789",
  "gene": "UniProtKB:Q06136",
  "gene_symbol": "KDSR",
  "term_label": "endoplasmic reticulum membrane"
}